activation of transmembrane receptor protein tyrosine kinase activity [GO:0007171] (biological process) Sources: GOC:dph, GOC:tb Also known as: transmembrane receptor protein tyrosine kinase activation, transmembrane receptor protein tyrosine kinase dimerization Relationships: is a type of activation of protein kinase activity [GO:0032147]; is_a protein-containing complex assembly [GO:0065003]; is part of cell surface receptor protein tyrosine kinase signaling pathway [GO:0007169] Definition: Any process that initiates the activity of the inactive transmembrane receptor protein tyrosine kinase activity.